{
  "gene_symbol": "FCAR",
  "term_label": "immune receptor activity",
  "gene_name": "Immunoglobulin alpha Fc receptor",
  "term_id": "GO:0140375",
  "gene": "UniProtKB:P24071"
}